{
  "term_label": "positive regulation of transcription elongation by RNA polymerase II",
  "term_id": "GO:0032968",
  "gene": "UniProtKB:O00472",
  "gene_symbol": "ELL2",
  "gene_name": "RNA polymerase II elongation factor ELL2"
}